nucleoside monophosphate phosphorylation [GO:0046940] (biological process) Relationships: is a type of nucleoside monophosphate metabolic process [GO:0009123]; is a type of nucleotide biosynthetic process [GO:0009165] Subtypes: AMP phosphorylation [GO:0006756], dAMP phosphorylation [GO:0061565], CMP phosphorylation [GO:0061566], dCMP phosphorylation [GO:0061567] Sources: GOC:ai Definition: The process of introducing one or more phosphate groups into a nucleoside monophosphate to produce a polyphosphorylated nucleoside.